{
  "term_label": "transcription coregulator activity",
  "gene_symbol": "SUPT20H",
  "gene": "UniProtKB:Q8NEM7",
  "gene_name": "Transcription factor SPT20 homolog",
  "term_id": "GO:0003712"
}